{
  "term_id": "GO:0006355",
  "term_label": "regulation of DNA-templated transcription",
  "gene_symbol": "ZNF460",
  "gene": "UniProtKB:Q14592",
  "gene_name": "Zinc finger protein 460"
}